{
  "gene_name": "Neuronal acetylcholine receptor subunit alpha-4",
  "gene_symbol": "CHRNA4",
  "term_label": "synapse",
  "gene": "UniProtKB:P43681",
  "term_id": "GO:0045202"
}